{
  "term_id": "GO:0031982",
  "term_label": "vesicle",
  "gene": "UniProtKB:P16442",
  "gene_name": "Histo-blood group ABO system transferase",
  "gene_symbol": "ABO"
}